{
  "gene_symbol": "TUBB4A",
  "term_id": "GO:0000226",
  "gene_name": "Tubulin beta-4A chain",
  "gene": "UniProtKB:P04350",
  "term_label": "microtubule cytoskeleton organization"
}